{
  "gene_symbol": "ANKRD54",
  "gene_name": "Ankyrin repeat domain-containing protein 54",
  "term_id": "GO:0005634",
  "gene": "UniProtKB:Q6NXT1",
  "term_label": "nucleus"
}